{
  "gene_name": "RING finger protein 141",
  "term_id": "GO:0051865",
  "term_label": "protein autoubiquitination",
  "gene_symbol": "RNF141",
  "gene": "UniProtKB:Q8WVD5"
}